rhodopsin metabolic process [GO:0046154] (biological process) Relationships: is_a protein metabolic process [GO:0019538]; is a type of eye pigment metabolic process [GO:0042441] Also known as: rhodopsin metabolism Definition: The chemical reactions and pathways involving rhodopsin, a brilliant purplish-red, light-sensitive visual pigment found in the rod cells of the retinas. Sources: ISBN:0198506732 Subtypes: rhodopsin biosynthetic process [GO:0016063]